node of Ranvier [GO:0033268] (cellular component) Relationships: is_a cellular anatomical structure [GO:0110165]; BFO_0000050 main axon [GO:0044304] Sources: GOC:mh Also known as: node of Ranvier axon Definition: An axon part that is a gap in the myelin where voltage-gated sodium channels cluster and saltatory conduction is executed.